{
  "term_id": "GO:1902358",
  "term_label": "sulfate transmembrane transport",
  "gene_name": "Sodium-independent sulfate anion transporter",
  "gene_symbol": "SLC26A11",
  "gene": "UniProtKB:Q86WA9"
}